{
  "gene": "UniProtKB:O43396",
  "gene_name": "Thioredoxin-like protein 1",
  "term_label": "protein-disulfide reductase activity",
  "term_id": "GO:0015035",
  "gene_symbol": "TXNL1"
}